{
  "gene_symbol": "MORC2",
  "term_label": "nucleus",
  "gene": "UniProtKB:Q9Y6X9",
  "gene_name": "ATPase MORC2",
  "term_id": "GO:0005634"
}